{
  "gene": "UniProtKB:Q9Y234",
  "gene_name": "Lipoyltransferase 1, mitochondrial",
  "gene_symbol": "LIPT1",
  "term_id": "GO:0017118",
  "term_label": "lipoyltransferase activity"
}